{
  "gene_symbol": "USP17L4",
  "term_label": "regulation of apoptotic process",
  "gene_name": "Inactive ubiquitin carboxyl-terminal hydrolase 17-like protein 4",
  "gene": "UniProtKB:A6NCW7",
  "term_id": "GO:0042981"
}